symbiont-mediated activation of host G protein-coupled receptor signal transduction [GO:0141104] (biological process) Relationships: is a type of symbiont-mediated activation of host signal transduction pathway [GO:0052028]; is a type of GO:0075118 References: PMID:15963708, PMID:18978047, PMID:25332123 Definition: A process in which a symbiont initiates, promotes, or enhances a G protein-coupled receptor signal transduction pathway in the host organism. The host is defined as the larger of the organisms involved in a symbiotic interaction.